mRNA editing complex [GO:0045293] (cellular component) Subtypes: apolipoprotein B mRNA editing enzyme complex [GO:0030895], GO:0031019, plastid mRNA editing complex [GO:0031020] References: PMID:11564867, PMID:12139607, PMID:24316715 Relationships: is a type of catalytic complex [GO:1902494] Definition: A protein complex that posttranscriptionally catalyzes insertion, deletion or substitution of nucleotides at multiple sites within nascent mRNA transcripts to produce mature mRNAs in eukaryotes. Also known as: editosome